{
  "term_id": "UNKNOWN:0003",
  "gene_symbol": "PSTK",
  "gene_name": "L-seryl-tRNA(Sec) kinase",
  "term_label": "Unknown cellular component",
  "gene": "UniProtKB:Q8IV42"
}